{
  "term_label": "monoatomic cation transmembrane transport",
  "gene_symbol": "TRPM7",
  "gene_name": "Transient receptor potential cation channel subfamily M member 7",
  "gene": "UniProtKB:Q96QT4",
  "term_id": "GO:0098655"
}